{
  "gene_name": "Uncharacterized protein C3orf38",
  "term_label": "Unknown molecular function",
  "gene_symbol": "C3orf38",
  "term_id": "UNKNOWN:0001",
  "gene": "UniProtKB:Q5JPI3"
}